regulation of seed dormancy process [GO:2000033] (biological process) Relationships: is_a regulation of seed maturation [GO:2000034]; regulates seed dormancy process [GO:0010162] Sources: GOC:obol, GOC:pr, ISBN:9781405139830 Subtypes: negative regulation of seed dormancy process [GO:1902039], GO:1902040 Also known as: regulation of seed dormancy Definition: Any process that modulates the frequency, rate or extent of seed dormancy process.